{
  "term_label": "Unknown biological process",
  "gene_symbol": "RPS6KC1",
  "gene": "UniProtKB:Q96S38",
  "term_id": "UNKNOWN:0002",
  "gene_name": "Ribosomal protein S6 kinase delta-1"
}